{
  "term_label": "chromatin binding",
  "term_id": "GO:0003682",
  "gene_symbol": "SAMD11",
  "gene": "UniProtKB:Q96NU1",
  "gene_name": "Sterile alpha motif domain-containing protein 11"
}